hemidesmosome assembly [GO:0031581] (biological process) References: PMID:15983403 Sources: GOC:dgh Relationships: is a type of cell-substrate junction assembly [GO:0007044] Definition: Assembly of hemidesmosomes, integrin-containing protein complexes that bind to laminin in the basal lamina. Hemidesmosomes form the contact between the basal surface of epithelial cells and the underlying basal lamina.